{
  "gene_name": "Olfactory receptor 51I2",
  "term_label": "plasma membrane",
  "gene": "UniProtKB:Q9H344",
  "gene_symbol": "OR51I2",
  "term_id": "GO:0005886"
}